{
  "term_id": "GO:0005886",
  "gene_name": "Putative olfactory receptor 1F12P",
  "gene": "UniProtKB:Q8NHA8",
  "term_label": "plasma membrane",
  "gene_symbol": "OR1F12P"
}